{
  "term_id": "GO:0005886",
  "term_label": "plasma membrane",
  "gene": "UniProtKB:Q7RTP6",
  "gene_name": "[F-actin]-monooxygenase MICAL3",
  "gene_symbol": "MICAL3"
}